FAD transmembrane transporter activity [GO:0015230] (molecular function) Definition: Enables the directed movement of flavin-adenine dinucleotide (FAD) from one side of a membrane to the other. FAD forms the coenzyme of the prosthetic group of various flavoprotein oxidoreductase enzymes, in which it functions as an electron acceptor by being reversibly converted to its reduced form. Sources: ISBN:0198506732 Also known as: FAD transporter activity, flavin adenine dinucleotide transmembrane transporter activity, flavin-adenine dinucleotide transmembrane transporter activity, FAD carrier activity, flavin adenine dinucleotide carrier activity, flavin-adenine dinucleotide carrier activity Relationships: is a type of nucleotide transmembrane transporter activity [GO:0015215]; is part of GO:0035350